{
  "term_id": "GO:0005634",
  "term_label": "nucleus",
  "gene_symbol": "SMYD2",
  "gene_name": "N-lysine methyltransferase SMYD2",
  "gene": "UniProtKB:Q9NRG4"
}